disseminated nephrocyte differentiation [GO:0061322] (biological process) Definition: The process in which a relatively unspecialized cell acquires the specialized structural and/or functional features of a disseminated nephrocyte. A disseminated nephrocyte is an insect renal cell that filters hemolymph and is found at scattered locations in the fat body or other tissues. Differentiation includes the processes involved in commitment of a cell to a specific fate and its subsequent development to the mature state. Relationships: is a type of nephrocyte differentiation [GO:0061319] Sources: CL:0002524, GOC:19783135, GOC:dph, GOC:mtg_kidney_jan10